{
  "term_id": "GO:0000122",
  "gene": "UniProtKB:Q9Y543",
  "gene_name": "Transcription factor HES-2",
  "gene_symbol": "HES2",
  "term_label": "negative regulation of transcription by RNA polymerase II"
}